activation of blood coagulation via clotting cascade [GO:0002543] (biological process) Relationships: is a type of positive regulation of blood coagulation [GO:0030194]; BFO_0000050 acute inflammatory response [GO:0002526] Sources: GOC:jal, ISBN:0781735149 Definition: Any process that initiates the clotting cascade of blood coagulation, a cascade of plasma enzymes that is triggered following damage to blood vessels, leading to formation of a clot. Also known as: activation of clotting cascade